{
  "term_label": "calcium ion binding",
  "gene": "UniProtKB:Q13586",
  "gene_name": "Stromal interaction molecule 1",
  "term_id": "GO:0005509",
  "gene_symbol": "STIM1"
}